vestibulocochlear nerve structural organization [GO:0021649] (biological process) Sources: GOC:cls, GOC:dgh, GOC:dph, GOC:jid, GO_REF:0000021 Relationships: is a type of cranial nerve structural organization [GO:0021604]; is part of vestibulocochlear nerve morphogenesis [GO:0021648] Definition: The process that contributes to the act of creating the structural organization of the vestibulocochlear nerve. This process pertains to the physical shaping of a rudimentary structure. This sensory nerve innervates the membranous labyrinth of the inner ear. The vestibular branch innervates the vestibular apparatus that senses head position changes relative to gravity. The auditory branch innervates the cochlear duct, which is connected to the three bony ossicles which transduce sound waves into fluid movement in the cochlea. Also known as: vestibulocochlear nerve structural organisation, CN VII structural organization